fumigermin biosynthetic process [GO:0140446] (biological process) Relationships: is a type of GO:0030639; is a type of lactone biosynthetic process [GO:1901336] Definition: The chemical reactions and pathways resulting in the formation of fumigermin, an alpha-pyrone secondary metabolite found in some species of fungi such as Aspergillus fumigatus. Also known as: fumigermin anabolism, fumigermin biosynthesis, fumigermin formation, fumigermin synthesis References: PMID:32083553